{
  "gene_symbol": "CBLN2",
  "term_label": "synapse",
  "term_id": "GO:0045202",
  "gene": "UniProtKB:Q8IUK8",
  "gene_name": "Cerebellin-2"
}